{
  "gene": "UniProtKB:Q6P4Q7",
  "gene_symbol": "CNNM4",
  "term_id": "GO:0015081",
  "gene_name": "Metal transporter CNNM4",
  "term_label": "sodium ion transmembrane transporter activity"
}